halohydrin hydrogen-halide-lyase activity [GO:0019181] (molecular function) References: PMID:8017917 Definition: Catalysis of the reaction: a halohydrin = an epoxide + a hydrogen halide. Relationships: is a type of GO:0016848